cellular response to dehydroepiandrosterone [GO:1903495] (biological process) Relationships: is a type of cellular response to lipid [GO:0071396]; is_a cellular response to alcohol [GO:0097306]; is a type of cellular response to ketone [GO:1901655]; is a type of response to dehydroepiandrosterone [GO:1903494] References: PMID:3585228 Sources: GOC:TermGenie, GOC:mr, GO_REF:0000071 Definition: Any process that results in a change in state or activity of a cell (in terms of movement, secretion, enzyme production, gene expression, etc.) as a result of a dehydroepiandrosterone stimulus.